{
  "term_label": "eukaryotic initiation factor 4E binding",
  "gene": "UniProtKB:O60516",
  "term_id": "GO:0008190",
  "gene_name": "Eukaryotic translation initiation factor 4E-binding protein 3",
  "gene_symbol": "EIF4EBP3"
}